{
  "gene": "UniProtKB:Q9UNY4",
  "gene_symbol": "TTF2",
  "term_label": "nucleus",
  "gene_name": "Transcription termination factor 2",
  "term_id": "GO:0005634"
}